{
  "gene_name": "E3 ubiquitin-protein ligase MIB1",
  "term_label": "ubiquitin protein ligase activity",
  "gene": "UniProtKB:Q86YT6",
  "term_id": "GO:0061630",
  "gene_symbol": "MIB1"
}